cellular response to starvation [GO:0009267] (biological process) Sources: GOC:jl Definition: Any process that results in a change in state or activity of a cell (in terms of movement, secretion, enzyme production, gene expression, etc.) as a result of deprivation of nourishment. Subtypes: cellular response to nitrogen starvation [GO:0006995], cellular response to sulfate starvation [GO:0009970], cellular response to iron ion starvation [GO:0010106], cellular response to magnesium starvation [GO:0010350], GO:0010438, GO:0015968, GO:0016036, aggregation involved in sorocarp development [GO:0031152], cellular response to amino acid starvation [GO:0034198], GO:0034224, cellular response to copper ion starvation [GO:0035874], cellular response to inositol starvation [GO:0036110], cellular response to adenine starvation [GO:0036223], cellular response to vitamin B1 starvation [GO:0036225], cellular response to glucose starvation [GO:0042149], cellular response to sucrose starvation [GO:0043617], cellular response to potassium ion starvation [GO:0051365], GO:0072732, cellular response to boron-containing substance deprivation [GO:0080169], cellular response to biotin starvation [GO:1990383] Relationships: is a type of cellular response to nutrient levels [GO:0031669]; is_a cellular response to stress [GO:0033554]; is a type of response to starvation [GO:0042594]